{
  "term_label": "regulation of iron ion transport",
  "gene_name": "Hereditary hemochromatosis protein",
  "gene_symbol": "HFE",
  "term_id": "GO:0034756",
  "gene": "UniProtKB:Q30201"
}